{
  "term_label": "regulation of transcription by RNA polymerase II",
  "gene_symbol": "ZNF580",
  "gene": "UniProtKB:Q9UK33",
  "term_id": "GO:0006357",
  "gene_name": "Zinc finger protein 580"
}